{
  "term_label": "vesicle-mediated transport",
  "gene_symbol": "AP1S3",
  "term_id": "GO:0016192",
  "gene_name": "AP-1 complex subunit sigma-3",
  "gene": "UniProtKB:Q96PC3"
}